{
  "gene_symbol": "PLBD1",
  "term_label": "Unknown biological process",
  "gene_name": "Phospholipase B-like 1",
  "term_id": "UNKNOWN:0002",
  "gene": "UniProtKB:Q6P4A8"
}